{
  "gene_name": "ARF GTPase-activating protein GIT2",
  "gene": "UniProtKB:Q14161",
  "term_id": "GO:0007420",
  "gene_symbol": "GIT2",
  "term_label": "brain development"
}